{
  "term_label": "Unknown biological process",
  "gene": "UniProtKB:A4D2B0",
  "gene_name": "Metallo-beta-lactamase domain-containing protein 1",
  "term_id": "UNKNOWN:0002",
  "gene_symbol": "MBLAC1"
}